diphthine synthase activity [GO:0004164] (molecular function) Also known as: S-adenosyl-L-methionine:2-(3-carboxy-3-aminopropyl)-L-histidine methyltransferase activity, S-adenosyl-L-methionine:elongation factor 2 methyltransferase activity, diphthine methyltransferase activity Relationships: is a type of protein methyltransferase activity [GO:0008276]; is a type of GO:0008757 Note: This activity is present in archae and produces the trimethylated product diphthine, which is converted into diphthamide by diphthine-ammonia ligase activity ; GO:0017178 (EC:6.3.1.14). Note that this is different from the eukaryotic enzyme diphthine methyl ester synthase activity ; GO:0141133 (EC:2.1.1.314), which produces diphthine methyl ester. References: PMID:15485916, PMID:20873788, PMID:3042777 Sources: RHEA:36415 Definition: Catalysis of the reaction: 2-[(3S)-amino-3-carboxypropyl]-L-histidyl-[translation elongation factor 2] + 3 S-adenosyl-L-methionine = diphthine-[translation elongation factor 2] + 3 H+ + 3 S-adenosyl-L-homocysteine.